{
  "term_label": "RNA polymerase II cis-regulatory region sequence-specific DNA binding",
  "gene": "UniProtKB:Q8TF32",
  "term_id": "GO:0000978",
  "gene_symbol": "ZNF431",
  "gene_name": "Zinc finger protein 431"
}